aldaric acid biosynthetic process [GO:0019578] (biological process) Subtypes: GO:0019393, galactarate biosynthetic process [GO:0046357] Relationships: is a type of dicarboxylic acid biosynthetic process [GO:0043650] Definition: The chemical reactions and pathways resulting in the formation of aldaric acid, any dicarboxylic acid formed by oxidation of by the terminal groups of an aldose to carboxyl group. Also known as: aldaric acid anabolism, aldaric acid biosynthesis, aldaric acid formation, aldaric acid synthesis Sources: ISBN:0198506732